{
  "term_id": "GO:0005765",
  "term_label": "lysosomal membrane",
  "gene_symbol": "DEPDC5",
  "gene_name": "GATOR complex protein DEPDC5",
  "gene": "UniProtKB:O75140"
}